{
  "gene_symbol": "EXOC3",
  "gene": "UniProtKB:O60645",
  "term_id": "GO:0051601",
  "term_label": "exocyst localization",
  "gene_name": "Exocyst complex component 3"
}